{
  "term_id": "GO:1990782",
  "gene_name": "Carcinoembryonic antigen-related cell adhesion molecule 4",
  "gene_symbol": "CEACAM4",
  "term_label": "protein tyrosine kinase binding",
  "gene": "UniProtKB:O75871"
}